{
  "gene_symbol": "OR51I1",
  "term_label": "plasma membrane",
  "gene_name": "Olfactory receptor 51I1",
  "term_id": "GO:0005886",
  "gene": "UniProtKB:Q9H343"
}